{
  "term_id": "UNKNOWN:0002",
  "gene_symbol": "TMEM72",
  "gene_name": "Transmembrane protein 72",
  "term_label": "Unknown biological process",
  "gene": "UniProtKB:A0PK05"
}